{
  "term_id": "GO:0007631",
  "gene": "UniProtKB:P49683",
  "gene_name": "Prolactin-releasing peptide receptor",
  "gene_symbol": "PRLHR",
  "term_label": "feeding behavior"
}